establishment of petal orientation [GO:0048498] (biological process) Relationships: is a type of GO:0048559; is part of GO:0048446 References: PMID:10572040 Sources: GOC:tb Definition: The process that determines the orientation of petals with reference to the central axis.